stem cell fate commitment [GO:0048865] (biological process) Sources: CL:0000034, GOC:isa_complete Relationships: is a type of GO:0045165; BFO_0000050 GO:0048863 Subtypes: neural crest cell fate commitment [GO:0014034] Definition: The process in which the developmental fate of a cell becomes restricted such that it will develop into a stem cell.